{
  "term_id": "GO:0101023",
  "gene_symbol": "TGFBR1",
  "gene": "UniProtKB:P36897",
  "gene_name": "TGF-beta receptor type-1",
  "term_label": "vascular endothelial cell proliferation"
}